{
  "gene": "UniProtKB:Q07666",
  "term_id": "GO:0005634",
  "gene_name": "KH domain-containing, RNA-binding, signal transduction-associated protein 1",
  "term_label": "nucleus",
  "gene_symbol": "KHDRBS1"
}